{
  "gene_name": "Stathmin",
  "gene": "UniProtKB:P16949",
  "term_id": "GO:0031110",
  "term_label": "regulation of microtubule polymerization or depolymerization",
  "gene_symbol": "STMN1"
}